{
  "gene": "UniProtKB:Q6PIZ9",
  "gene_symbol": "TRAT1",
  "gene_name": "T-cell receptor-associated transmembrane adapter 1",
  "term_id": "GO:0050862",
  "term_label": "positive regulation of T cell receptor signaling pathway"
}